{
  "gene": "UniProtKB:O60341",
  "term_label": "flavin adenine dinucleotide binding",
  "gene_name": "Lysine-specific histone demethylase 1A",
  "gene_symbol": "KDM1A",
  "term_id": "GO:0050660"
}